cytosolic aryl hydrocarbon receptor complex [GO:0034752] (cellular component) Relationships: is a type of aryl hydrocarbon receptor complex [GO:0034751]; is part of GO:0005829 References: PMID:7598497, PMID:8937476, PMID:9447995 Definition: An aryl hydrocarbon receptor complex found in the cytosol, in which the ligand-binding subunit AhR is not bound to ligand; consists of AhR, two molecules of HSP90, the protein kinase c-Src, and the immunophilin XAP2/AIP. Also known as: cytosolic AHRC, cytosolic AhR complex, 9S-cytosolic aryl hydrocarbon (Ah) receptor non-ligand activated complex